{
  "gene": "UniProtKB:O14983",
  "gene_name": "Sarcoplasmic_endoplasmic reticulum calcium ATPase 1",
  "gene_symbol": "ATP2A1",
  "term_id": "GO:0016020",
  "term_label": "membrane"
}